{
  "term_label": "negative regulation of transcription by RNA polymerase II",
  "gene_symbol": "SKOR1",
  "gene_name": "SKI family transcriptional corepressor 1",
  "gene": "UniProtKB:P84550",
  "term_id": "GO:0000122"
}